low-affinity sodium:dicarboxylate symporter activity [GO:0015361] (molecular function) Sources: TC:2.A.47.1.1 Definition: Enables the transfer of a solute or solutes from one side of a membrane to the other according to the reaction: dicarboxylate(out) + Na+(out) = dicarboxylate(in) + Na+(in). In low-affinity transport the transporter is able to bind the solute only if it is present at very high concentrations. Also known as: low affinity sodium:dicarboxylate cotransporter activity, low affinity sodium:dicarboxylate symporter activity Relationships: is a type of sodium:dicarboxylate symporter activity [GO:0017153]